{
  "term_label": "growth factor activity",
  "gene": "UniProtKB:P0DML2",
  "gene_name": "Chorionic somatomammotropin hormone 1",
  "gene_symbol": "CSH1",
  "term_id": "GO:0008083"
}